{
  "term_id": "GO:0006357",
  "gene_symbol": "ZBTB8A",
  "gene": "UniProtKB:Q96BR9",
  "term_label": "regulation of transcription by RNA polymerase II",
  "gene_name": "Zinc finger and BTB domain-containing protein 8A"
}